protein secretion [GO:0009306] (biological process) Sources: GOC:ai Relationships: is a type of protein transport [GO:0015031]; is a type of secretion by cell [GO:0032940]; is a type of establishment of protein localization to extracellular region [GO:0035592]; is a type of GO:0071692 Subtypes: renin secretion into blood stream [GO:0002001], protein secretion by the type II secretion system [GO:0015628], insulin secretion [GO:0030073], protein secretion by the type I secretion system [GO:0030253], GO:0030254, protein secretion by the type IV secretion system [GO:0030255], protein secretion by the type VI secretion system [GO:0033103], secretion of lysosomal enzymes [GO:0033299], GO:0036394, BMP secretion [GO:0038055], protein secretion by the type VII secretion system [GO:0044315], protein secretion by the type V secretion system [GO:0046819], Wnt protein secretion [GO:0061355], adiponectin secretion [GO:0070162], prolactin secretion [GO:0070459], protein secretion by platelet [GO:0070560], basolateral protein secretion [GO:0110010], protein secretion by the type IX secretion system [GO:0160303], pancreatic trypsinogen secretion [GO:1990747], matrix metallopeptidase secretion [GO:1990773] Regulation: regulated by GO:0050708; negatively regulated by negative regulation of protein secretion [GO:0050709]; positively regulated by GO:0050714 Definition: The controlled release of proteins from a cell. Also known as: glycoprotein secretion, protein secretion during cell fate commitment, protein secretion resulting in cell fate commitment